phosphomevalonate decarboxylase activity [GO:0090710] (molecular function) References: PMID:24375100 Sources: RHEA:40955 Definition: Catalysis of the reaction: (R)-5-phosphomevalonate + ATP = ADP + CO2 + isopentenyl phosphate + phosphate. Relationships: is a type of carboxy-lyase activity [GO:0016831]